{
  "gene": "UniProtKB:O75711",
  "term_id": "UNKNOWN:0001",
  "term_label": "Unknown molecular function",
  "gene_name": "Scrapie-responsive protein 1",
  "gene_symbol": "SCRG1"
}